{
  "gene_name": "Potassium channel subfamily K member 13",
  "gene": "UniProtKB:Q9HB14",
  "term_label": "plasma membrane",
  "term_id": "GO:0005886",
  "gene_symbol": "KCNK13"
}